negative regulation of pyroptotic inflammatory response [GO:0160028] (biological process) Definition: Any process that decreases the frequency, rate or extent of a pyroptotic inflammatory response. References: PMID:34637033 Also known as: negative regulation of pyroptosis Relationships: is a type of negative regulation of inflammatory response [GO:0050728]; negatively regulates pyroptotic inflammatory response [GO:0070269]